{
  "term_id": "GO:0009755",
  "gene_name": "Nuclear receptor subfamily 1 group D member 2",
  "term_label": "hormone-mediated signaling pathway",
  "gene": "UniProtKB:Q14995",
  "gene_symbol": "NR1D2"
}